box H/ACA snoRNA binding [GO:0034513] (molecular function) Sources: GOC:mah Relationships: is a type of snoRNA binding [GO:0030515] Definition: Binding to a box H/ACA small nucleolar RNA.